{
  "term_id": "UNKNOWN:0001",
  "gene_name": "Liprin-beta-1",
  "term_label": "Unknown molecular function",
  "gene_symbol": "PPFIBP1",
  "gene": "UniProtKB:Q86W92"
}